{
  "gene_symbol": "CD55",
  "term_label": "Unknown molecular function",
  "gene_name": "Complement decay-accelerating factor",
  "gene": "UniProtKB:P08174",
  "term_id": "UNKNOWN:0001"
}